microtubule minus-end binding [GO:0051011] (molecular function) Relationships: is a type of microtubule binding [GO:0008017] References: PMID:14557818, PMID:14614826 Sources: GOC:ai Definition: Binding to the minus end of a microtubule.